{
  "gene": "UniProtKB:Q6NSJ0",
  "gene_symbol": "MYORG",
  "term_id": "UNKNOWN:0001",
  "term_label": "Unknown molecular function",
  "gene_name": "Myogenesis-regulating glycosidase"
}